signal transduction in response to DNA damage [GO:0042770] (biological process) Definition: A cascade of processes induced by the detection of DNA damage within a cell. Subtypes: DNA damage checkpoint signaling [GO:0000077], DNA damage response, signal transduction by p53 class mediator [GO:0030330], DNA damage response, signal transduction resulting in transcription [GO:0042772] Also known as: DNA damage response, signal transduction, response to DNA damage stimulus by intracellular signaling cascade, DNA damage induced protein phosphorylation Sources: GOC:go_curators Relationships: is a type of DNA damage response [GO:0006974]; is a type of intracellular signal transduction [GO:0035556]